regulation of protein complex stability [GO:0061635] (biological process) Sources: GOC:dph Relationships: is_a regulation of biological quality [GO:0065008] Definition: Any process that affects the structure and integrity of a protein complex by altering the likelihood of its assembly or disassembly.